{
  "term_label": "nucleus",
  "gene_name": "Zinc finger protein 276",
  "term_id": "GO:0005634",
  "gene": "UniProtKB:Q8N554",
  "gene_symbol": "ZNF276"
}